{
  "gene_name": "Transmembrane protein 215",
  "term_id": "UNKNOWN:0001",
  "term_label": "Unknown molecular function",
  "gene_symbol": "TMEM215",
  "gene": "UniProtKB:Q68D42"
}